{
  "gene_symbol": "PICALM",
  "term_label": "clathrin-coated vesicle",
  "gene": "UniProtKB:Q13492",
  "term_id": "GO:0030136",
  "gene_name": "Phosphatidylinositol-binding clathrin assembly protein"
}